{
  "term_label": "ERAD pathway",
  "gene_name": "Ubiquilin-2",
  "term_id": "GO:0036503",
  "gene": "UniProtKB:Q9UHD9",
  "gene_symbol": "UBQLN2"
}